nucleotide transmembrane transporter activity [GO:0015215] (molecular function) Relationships: is a type of organophosphate ester transmembrane transporter activity [GO:0015605]; is a type of nucleobase-containing compound transmembrane transporter activity [GO:0015932]; is part of nucleotide transmembrane transport [GO:1901679] Definition: Enables the transfer of a nucleotide, any compound consisting of a nucleoside that is esterified with (ortho)phosphate, from one side of a membrane to the other. Sources: ISBN:0198506732 Subtypes: purine nucleotide transmembrane transporter activity [GO:0015216], GO:0015218, GO:0015230, nicotinamide mononucleotide transmembrane transporter activity [GO:0015663], deoxynucleotide transmembrane transporter activity [GO:0030233], FMN transmembrane transporter activity [GO:0044610]